{
  "gene": "UniProtKB:Q9H239",
  "term_id": "GO:0004222",
  "gene_name": "Matrix metalloproteinase-28",
  "term_label": "metalloendopeptidase activity",
  "gene_symbol": "MMP28"
}